{
  "gene_symbol": "CTNNB1",
  "gene": "UniProtKB:P35222",
  "term_id": "GO:0045944",
  "gene_name": "Catenin beta-1",
  "term_label": "positive regulation of transcription by RNA polymerase II"
}